{
  "gene": "UniProtKB:Q9BYG3",
  "gene_symbol": "NIFK",
  "gene_name": "MKI67 FHA domain-interacting nucleolar phosphoprotein",
  "term_id": "GO:0003723",
  "term_label": "RNA binding"
}